{
  "gene_name": "Disabled homolog 2",
  "gene_symbol": "DAB2",
  "gene": "UniProtKB:P98082",
  "term_id": "GO:0090090",
  "term_label": "negative regulation of canonical Wnt signaling pathway"
}